{
  "term_id": "GO:0003785",
  "gene": "UniProtKB:O14604",
  "gene_name": "Thymosin beta-4, Y-chromosomal",
  "term_label": "actin monomer binding",
  "gene_symbol": "TMSB4Y"
}